facial nerve structural organization [GO:0021612] (biological process) Also known as: facial nerve structural organisation, CN VII structural organization Definition: The process that contributes to the act of creating the structural organization of the facial nerve. This process pertains to the physical shaping of a rudimentary structure. This sensory and motor nerve supplies the muscles of facial expression and the expression and taste at the anterior two-thirds of the tongue. The principal branches are the superficial ophthalmic, buccal, palatine and hyomandibular. The main trunk synapses within pterygopalatine ganglion in the parotid gland and this ganglion then gives of nerve branches which supply the lacrimal gland and the mucous secreting glands of the nasal and oral cavities. Relationships: is_a cranial nerve structural organization [GO:0021604]; is part of facial nerve morphogenesis [GO:0021610] Sources: GOC:cls, GOC:dgh, GOC:dph, GOC:jid, GO_REF:0000021